L-tryptophan catabolic process [GO:0006569] (biological process) Sources: ISBN:0198547684 Relationships: is a type of GO:0006568; is a type of aromatic amino acid family catabolic process [GO:0009074]; is a type of indole-containing compound catabolic process [GO:0042436]; is a type of GO:0170035; is a type of proteinogenic amino acid catabolic process [GO:0170040] Also known as: tryptophan breakdown, tryptophan catabolism, tryptophan degradation, tryptophan catabolic process, using tryptophanase, tryptophan catabolism, using tryptophanase, tryptophan catabolic process Subtypes: L-tryptophan catabolic process to indole-3-acetate [GO:0019440], L-tryptophan catabolic process to kynurenine [GO:0019441], L-tryptophan catabolic process to acetyl-CoA [GO:0019442], GO:0019444 Definition: The chemical reactions and pathways resulting in the breakdown of L-tryptophan, the chiral amino acid 2-amino-3-(1H-indol-3-yl)propanoic acid.